response to UV-C [GO:0010225] (biological process) Definition: Any process that results in a change in state or activity of a cell or an organism (in terms of movement, secretion, enzyme production, gene expression, etc.) as a result of a UV-C radiation stimulus. UV-C radiation (UV-C light) spans the wavelengths 100 to 280 nm. Also known as: response to UV-C light stimulus, response to UV-C radiation stimulus, response to UVC light stimulus, response to UVC radiation stimulus, response to germicidal ultraviolet light stimulus, response to germicidal ultraviolet radiation stimulus, response to shortwave ultraviolet light stimulus, response to shortwave ultraviolet radiation stimulus Subtypes: cellular response to UV-C [GO:0071494] Sources: GOC:tb Relationships: is a type of response to UV [GO:0009411]